{
  "gene_name": "Dematin",
  "term_label": "actin cytoskeleton",
  "gene_symbol": "DMTN",
  "gene": "UniProtKB:Q08495",
  "term_id": "GO:0015629"
}